{
  "gene_name": "Guanine nucleotide-binding protein subunit alpha-11",
  "term_id": "GO:0005737",
  "gene": "UniProtKB:P29992",
  "term_label": "cytoplasm",
  "gene_symbol": "GNA11"
}